{
  "gene": "UniProtKB:Q9ULW5",
  "term_id": "GO:0005768",
  "gene_symbol": "RAB26",
  "term_label": "endosome",
  "gene_name": "Ras-related protein Rab-26"
}